{
  "term_label": "RNA polymerase II cis-regulatory region sequence-specific DNA binding",
  "gene_symbol": "SREBF1",
  "gene": "UniProtKB:P36956",
  "term_id": "GO:0000978",
  "gene_name": "Sterol regulatory element-binding protein 1"
}